{
  "term_id": "UNKNOWN:0003",
  "gene_symbol": "LYRM1",
  "term_label": "Unknown cellular component",
  "gene_name": "LYR motif-containing protein 1",
  "gene": "UniProtKB:O43325"
}